plus-end-directed organelle transport along microtubule [GO:0072386] (biological process) Definition: The directed movement of an organelle towards the plus end of a microtubule, mediated by motor proteins. This process begins with the attachment of an organelle to a microtubule, and ends when the organelle reaches its final destination. Subtypes: GO:0072383 Relationships: is a type of organelle transport along microtubule [GO:0072384] Sources: GOC:BHF, GOC:mah Also known as: microtubule plus-end-directed organelle localization, microtubule plus-end-directed organelle distribution